{
  "gene": "UniProtKB:Q92547",
  "term_label": "mitotic G2 DNA damage checkpoint signaling",
  "gene_symbol": "TOPBP1",
  "term_id": "GO:0007095",
  "gene_name": "DNA topoisomerase 2-binding protein 1"
}